{
  "gene_name": "Histone deacetylase 4",
  "gene_symbol": "HDAC4",
  "term_id": "GO:0000118",
  "term_label": "histone deacetylase complex",
  "gene": "UniProtKB:P56524"
}